{
  "term_label": "nucleus",
  "gene": "UniProtKB:O15090",
  "term_id": "GO:0005634",
  "gene_name": "Zinc finger protein 536",
  "gene_symbol": "ZNF536"
}